activation of innate immune response [GO:0002218] (biological process) Definition: Any process that initiates an innate immune response. Innate immune responses are defense responses mediated by germline encoded components that directly recognize components of potential pathogens. Examples of this process include activation of the hypersensitive response of Arabidopsis thaliana and activation of any NOD or TLR signaling pathway in vertebrate species. References: PMID:15199967, PMID:16177805 Sources: GOC:add, GOC:mtg_sensu, GO_REF:0000022, ISBN:0781735149 Subtypes: GO:0002758, GO:0009864, induced systemic resistance, ethylene mediated signaling pathway [GO:0009866] Relationships: is a type of GO:0002253; is a type of positive regulation of innate immune response [GO:0045089]